{
  "term_label": "Unknown biological process",
  "gene_symbol": "TMA7B",
  "term_id": "UNKNOWN:0002",
  "gene": "UniProtKB:A0A024R1R8",
  "gene_name": "Translation machinery-associated protein 7B"
}